{
  "gene_name": "LETM1 domain-containing protein 1",
  "term_label": "Unknown biological process",
  "gene_symbol": "LETMD1",
  "gene": "UniProtKB:Q6P1Q0",
  "term_id": "UNKNOWN:0002"
}